{
  "gene_name": "Iron-sulfur clusters transporter ABCB7, mitochondrial",
  "gene_symbol": "ABCB7",
  "term_label": "mitochondrial inner membrane",
  "term_id": "GO:0005743",
  "gene": "UniProtKB:O75027"
}